{
  "gene_symbol": "FAM215A",
  "gene_name": "Uncharacterized protein FAM215A",
  "gene": "UniProtKB:Q9Y5M1",
  "term_label": "Unknown molecular function",
  "term_id": "UNKNOWN:0001"
}